{
  "term_label": "signaling receptor binding",
  "term_id": "GO:0005102",
  "gene_symbol": "CD276",
  "gene": "UniProtKB:Q5ZPR3",
  "gene_name": "CD276 antigen"
}